G protein-coupled opioid receptor signaling pathway [GO:0038003] (biological process) Definition: A G protein-coupled receptor signaling pathway initiated by an opioid binding to its receptor on the surface of a target cell, and ending with the regulation of a downstream cellular process. References: PMID:20494127 Sources: GOC:bf Also known as: opioid receptor signaling pathway, opioid receptor signalling pathway Relationships: is a type of GO:0007186 Subtypes: GO:0031635 Regulation: regulated by regulation of opioid receptor signaling pathway [GO:2000474]; negatively regulated by negative regulation of opioid receptor signaling pathway [GO:2000475]; positively regulated by positive regulation of opioid receptor signaling pathway [GO:2000476]